regulation of protein processing [GO:0070613] (biological process) Also known as: regulation of protein maturation by peptide bond cleavage Relationships: is a type of GO:0030162; is a type of regulation of protein maturation [GO:1903317]; regulates GO:0016485 Subtypes: regulation of plasminogen activation [GO:0010755], GO:0010954, negative regulation of protein processing [GO:0010955], regulation of peptide hormone processing [GO:0060568], regulation of protein processing involved in protein targeting to mitochondrion [GO:1903216], GO:1903921 Sources: GOC:mah Definition: Any process that modulates the frequency, rate or extent of protein processing, a protein maturation process achieved by the cleavage of a peptide bond or bonds within a protein.